{
  "gene_name": "Zinc finger protein 853",
  "term_label": "DNA-binding transcription factor activity, RNA polymerase II-specific",
  "term_id": "GO:0000981",
  "gene": "UniProtKB:P0CG23",
  "gene_symbol": "ZNF853"
}